{
  "gene_name": "Olfactory receptor 10Q1",
  "term_id": "UNKNOWN:0003",
  "term_label": "Unknown cellular component",
  "gene": "UniProtKB:Q8NGQ4",
  "gene_symbol": "OR10Q1"
}